{
  "gene_name": "Serine_threonine-protein kinase MRCK beta",
  "term_label": "actomyosin structure organization",
  "term_id": "GO:0031032",
  "gene": "UniProtKB:Q9Y5S2",
  "gene_symbol": "CDC42BPB"
}